determination of stimulus intensity [GO:0050889] (biological process) Relationships: is a type of sensory processing [GO:0050893] Sources: ISBN:0721619908 Definition: The determination of the perceived strength of a sensory stimulus.